{
  "term_id": "UNKNOWN:0002",
  "gene": "UniProtKB:Q8IYM2",
  "gene_symbol": "SLFN12",
  "gene_name": "Ribonuclease SLFN12",
  "term_label": "Unknown biological process"
}